{
  "term_id": "GO:0005737",
  "gene_name": "Tripartite motif-containing protein 54",
  "gene": "UniProtKB:Q9BYV2",
  "term_label": "cytoplasm",
  "gene_symbol": "TRIM54"
}